{
  "gene_name": "Kinesin-like protein KIF2C",
  "term_label": "microtubule binding",
  "gene": "UniProtKB:Q99661",
  "gene_symbol": "KIF2C",
  "term_id": "GO:0008017"
}